{
  "gene_name": "Glycerophosphodiester phosphodiesterase 1",
  "term_label": "glycerophosphodiester phosphodiesterase activity",
  "gene": "UniProtKB:Q9NZC3",
  "gene_symbol": "GDE1",
  "term_id": "GO:0008889"
}